{
  "gene": "UniProtKB:O75037",
  "gene_symbol": "KIF21B",
  "term_id": "GO:0008017",
  "gene_name": "Kinesin-like protein KIF21B",
  "term_label": "microtubule binding"
}